{
  "gene": "UniProtKB:Q8N8P6",
  "term_id": "UNKNOWN:0002",
  "term_label": "Unknown biological process",
  "gene_name": "Putative uncharacterized protein FLJ39060",
  "gene_symbol": "Q8N8P6"
}